regulation of feeding behavior [GO:0060259] (biological process) Definition: Any process that modulates the rate, frequency or extent of the behavior associated with the intake of food. Subtypes: GO:0075329, regulation of eating behavior [GO:1903998], GO:2000252, positive regulation of feeding behavior [GO:2000253] Relationships: is a type of GO:0050795; regulates feeding behavior [GO:0007631] Also known as: regulation of feeding behaviour Sources: GOC:BHF, GOC:dph, GOC:tb